{
  "term_label": "plasma membrane",
  "gene_name": "Olfactory receptor 6X1",
  "gene_symbol": "OR6X1",
  "term_id": "GO:0005886",
  "gene": "UniProtKB:Q8NH79"
}